{
  "gene": "UniProtKB:Q14865",
  "gene_name": "AT-rich interactive domain-containing protein 5B",
  "gene_symbol": "ARID5B",
  "term_label": "nucleus",
  "term_id": "GO:0005634"
}